{
  "term_id": "GO:0033691",
  "gene_symbol": "SIGLEC10",
  "gene": "UniProtKB:Q96LC7",
  "term_label": "sialic acid binding",
  "gene_name": "Sialic acid-binding Ig-like lectin 10"
}